metanephric nephron tubule formation [GO:0072289] (biological process) Definition: The developmental process pertaining to the initial formation of a metanephric nephron tubule from unspecified parts. A metanephric nephron tubule is an epithelial tube that is part of a nephron in the metanephros. Sources: GOC:mtg_kidney_jan10 Relationships: is a type of GO:0072079; is a type of metanephric tubule formation [GO:0072174]; is part of metanephric nephron tubule morphogenesis [GO:0072282]